{
  "gene_name": "U6 snRNA-associated Sm-like protein LSm4",
  "term_id": "GO:0000932",
  "gene_symbol": "LSM4",
  "term_label": "P-body",
  "gene": "UniProtKB:Q9Y4Z0"
}